{
  "gene": "UniProtKB:Q9NZD4",
  "gene_name": "Alpha-hemoglobin-stabilizing protein",
  "term_id": "GO:0005737",
  "term_label": "cytoplasm",
  "gene_symbol": "AHSP"
}